palmitoyltransferase activity [GO:0016409] (molecular function) Definition: Catalysis of the transfer of a palmitoyl (CH3-[CH2]14-CO-) group to an acceptor molecule. Sources: GOC:ai Note: Note that this term should not be confused with 'palmitoleoyltransferase activity ; GO:1990698'. Relationships: is a type of acyltransferase activity, transferring groups other than amino-acyl groups [GO:0016747] Subtypes: O-palmitoyltransferase activity [GO:0016416], C-palmitoyltransferase activity [GO:0016454], protein-cysteine S-palmitoyltransferase activity [GO:0019706]